{
  "gene_symbol": "NEU2",
  "term_id": "GO:0004308",
  "gene_name": "Sialidase-2",
  "term_label": "exo-alpha-sialidase activity",
  "gene": "UniProtKB:Q9Y3R4"
}